{
  "term_label": "extracellular space",
  "gene_name": "Bone morphogenetic protein 10",
  "term_id": "GO:0005615",
  "gene_symbol": "BMP10",
  "gene": "UniProtKB:O95393"
}